{
  "gene_name": "RUN and FYVE domain-containing protein 2",
  "gene_symbol": "RUFY2",
  "gene": "UniProtKB:Q8WXA3",
  "term_id": "GO:0005737",
  "term_label": "cytoplasm"
}